response to ischemia [GO:0002931] (biological process) Definition: Any process that results in a change in state or activity of an organism (in terms of movement, secretion, enzyme production, gene expression, etc.) as a result of a inadequate blood supply. Sources: GOC:hjd Note: Ischemia always results in hypoxia; however, hypoxia can occur without ischemia. Relationships: is a type of response to stress [GO:0006950]